{
  "term_label": "Unknown molecular function",
  "gene": "UniProtKB:Q9NXH8",
  "gene_symbol": "TOR4A",
  "term_id": "UNKNOWN:0001",
  "gene_name": "Torsin-4A"
}